{
  "gene_name": "Epidermal growth factor receptor",
  "term_label": "plasma membrane",
  "gene_symbol": "EGFR",
  "term_id": "GO:0005886",
  "gene": "UniProtKB:P00533"
}